{
  "term_id": "GO:0003723",
  "gene_name": "Non-POU domain-containing octamer-binding protein",
  "gene_symbol": "NONO",
  "term_label": "RNA binding",
  "gene": "UniProtKB:Q15233"
}